{
  "gene_symbol": "NCKAP1",
  "term_label": "cell projection assembly",
  "term_id": "GO:0030031",
  "gene_name": "Nck-associated protein 1",
  "gene": "UniProtKB:Q9Y2A7"
}